chlamydospore septin filament array [GO:0032166] (cellular component) Relationships: is a type of septin filament array [GO:0032160] Definition: Arrays of septin filaments, or bars, found in a series of filamentous structures. Observed in the chlamydospore membrane during chlamydospore formation. References: PMID:16151244 Sources: GOC:krc